malonyltransferase activity [GO:0016420] (molecular function) Subtypes: S-malonyltransferase activity [GO:0016419], N-malonyltransferase activity [GO:0050735], GO:0050736 Definition: Catalysis of the transfer of a malonyl (HOOC-CH2-CO-) group to an acceptor molecule. Relationships: is a type of acyltransferase activity, transferring groups other than amino-acyl groups [GO:0016747] Sources: GOC:ai